{
  "gene_symbol": "NME2P1",
  "term_id": "UNKNOWN:0003",
  "gene": "UniProtKB:O60361",
  "term_label": "Unknown cellular component",
  "gene_name": "Putative nucleoside diphosphate kinase"
}